regulation of postsynapse to nucleus signaling pathway [GO:1905539] (biological process) Definition: Any process that modulates the frequency, rate or extent of postsynapse to nucleus signaling pathway. Sources: GOC:TermGenie, GO_REF:0000058, ISBN:9780071120005 Also known as: regulation of postsynaptic signaling to nucleus Relationships: is a type of regulation of signal transduction [GO:0009966]; regulates postsynapse to nucleus signaling pathway [GO:0099527]